{
  "term_id": "GO:0005737",
  "term_label": "cytoplasm",
  "gene_name": "Heat shock protein beta-7",
  "gene_symbol": "HSPB7",
  "gene": "UniProtKB:Q9UBY9"
}